positive regulation of intracellular mRNA localization [GO:1904582] (biological process) Also known as: positive regulation of establishment and maintenance of intracellular RNA localization, positive regulation of intracellular mRNA localisation, positive regulation of mRNA localization, intracellular, up regulation of establishment and maintenance of intracellular RNA localization, up regulation of intracellular mRNA localisation, up regulation of intracellular mRNA localization, up regulation of mRNA localization, intracellular, up-regulation of establishment and maintenance of intracellular RNA localization, up-regulation of intracellular mRNA localisation, up-regulation of intracellular mRNA localization, up-regulation of mRNA localization, intracellular, upregulation of establishment and maintenance of intracellular RNA localization, upregulation of intracellular mRNA localisation, upregulation of intracellular mRNA localization, upregulation of mRNA localization, intracellular, activation of establishment and maintenance of intracellular RNA localization, activation of intracellular mRNA localisation, activation of intracellular mRNA localization, activation of intracellular mRNA positioning, activation of mRNA localization, intracellular, activation of mRNA positioning, intracellular, positive regulation of intracellular mRNA positioning, positive regulation of mRNA positioning, intracellular, up regulation of intracellular mRNA positioning, up regulation of mRNA positioning, intracellular, up-regulation of intracellular mRNA positioning, up-regulation of mRNA positioning, intracellular, upregulation of intracellular mRNA positioning, upregulation of mRNA positioning, intracellular Relationships: is a type of positive regulation of biological process [GO:0048518]; is_a GO:1904580; positively regulates intracellular mRNA localization [GO:0008298] Subtypes: GO:0045854, positive regulation of pole plasm oskar mRNA localization [GO:0045856] Definition: Any process that activates or increases the frequency, rate or extent of intracellular mRNA localization. References: PMID:21471000 Sources: GOC:TermGenie, GO_REF:0000058